regulation of leukocyte activation [GO:0002694] (biological process) Sources: GOC:add Relationships: is a type of regulation of immune system process [GO:0002682]; is a type of regulation of cell activation [GO:0050865]; regulates leukocyte activation [GO:0045321] Subtypes: GO:0002695, GO:0002696, regulation of myeloid dendritic cell activation [GO:0030885], regulation of mast cell activation [GO:0033003], GO:0043030, regulation of lymphocyte activation [GO:0051249], regulation of neutrophil activation [GO:1902563], GO:1902566 Definition: Any process that modulates the frequency, rate, or extent of leukocyte activation. Also known as: regulation of immune cell activation, regulation of leucocyte activation